glucuronoside transport [GO:0015779] (biological process) Definition: The directed movement of glucuronosides into, out of or within a cell, or between cells, by means of some agent such as a transporter or pore. Glucuronosides are any compound formed by combination of glycosidic linkage of a hydroxy compound (e.g. an alcohol or a saccharide) with the anomeric carbon atom of glucuronate. Sources: GOC:ai Also known as: glucuronide transport Relationships: is a type of GO:1901656